{
  "gene_name": "Olfactory receptor 5G3",
  "gene_symbol": "OR5G3",
  "gene": "UniProtKB:P0C626",
  "term_id": "UNKNOWN:0003",
  "term_label": "Unknown cellular component"
}